{
  "gene": "UniProtKB:O15126",
  "term_id": "UNKNOWN:0001",
  "gene_name": "Secretory carrier-associated membrane protein 1",
  "gene_symbol": "SCAMP1",
  "term_label": "Unknown molecular function"
}